gamma-delta T cell receptor complex [GO:0042106] (CC) Definition: A T cell receptor complex in which the TCR heterodimer comprises gamma and delta chains, associated with the CD3 complex; recognizes antigen directly, without a requirement for processing and presentation by an MHC protein. Sources: GOC:mah, ISBN:0781735149 Relationships: is a type of T cell receptor complex [GO:0042101] Also known as: gamma-delta T lymphocyte receptor complex, gamma-delta T-cell receptor complex, gamma-delta T-lymphocyte receptor complex, gamma-delta TCR complex